{
  "gene_name": "Diphosphoinositol polyphosphate phosphohydrolase 2",
  "term_label": "diphosphoinositol-polyphosphate diphosphatase activity",
  "term_id": "GO:0008486",
  "gene": "UniProtKB:Q9NZJ9",
  "gene_symbol": "NUDT4"
}